{
  "gene_symbol": "ST6GALNAC6",
  "term_id": "GO:0009311",
  "term_label": "oligosaccharide metabolic process",
  "gene_name": "Alpha-N-acetylgalactosaminide alpha-2,6-sialyltransferase 6",
  "gene": "UniProtKB:Q969X2"
}